positive regulation of adenylate cyclase-inhibiting opioid receptor signaling pathway [GO:1900731] (biological process) Definition: Any process that activates or increases the frequency, rate or extent of adenylate cyclase-inhibiting opioid receptor signaling pathway. Relationships: is a type of regulation of adenylate cyclase-inhibiting opioid receptor signaling pathway [GO:1900729]; is a type of positive regulation of opioid receptor signaling pathway [GO:2000476]; positively regulates GO:0031635 Also known as: up regulation of adenylate cyclase-inhibiting opioid receptor signaling pathway, upregulation of adenylate cyclase-inhibiting opioid receptor signaling pathway, activation of adenylate cyclase-inhibiting opioid receptor signaling pathway, activation of opioid receptor-mediated adenylate cyclase inhibition References: PMID:17157995 Sources: GOC:TermGenie, GOC:sjw